negative regulation of single-strand break repair via homologous recombination [GO:1903111] (biological process) Also known as: down regulation of single-strand break repair via homologous recombination, down-regulation of single-strand break repair via homologous recombination, downregulation of single-strand break repair via homologous recombination, inhibition of single-strand break repair via homologous recombination Relationships: is a type of negative regulation of DNA recombination [GO:0045910]; is a type of GO:1903110; is a type of negative regulation of single strand break repair [GO:1903517]; negatively regulates single-strand break repair via homologous recombination [GO:1990396] References: PMID:24339919 Sources: GOC:TermGenie, GOC:bhm, GO_REF:0000058 Definition: Any process that stops, prevents or reduces the frequency, rate or extent of single-strand break repair via homologous recombination.